sesquiterpenoid biosynthetic process [GO:0016106] (biological process) Relationships: is a type of sesquiterpenoid metabolic process [GO:0006714]; is a type of GO:0016114 Also known as: sesquiterpenoid anabolism, sesquiterpenoid biosynthesis, sesquiterpenoid formation, sesquiterpenoid synthesis Sources: GOC:go_curators Subtypes: farnesol biosynthetic process [GO:0006715], juvenile hormone biosynthetic process [GO:0006718], abscisic acid biosynthetic process [GO:0009688], phaseic acid biosynthetic process [GO:0010379], vomitoxin biosynthetic process [GO:0106110], GO:0106210, GO:0140652, PR-toxin biosynthetic process [GO:0140875], GO:1901601, pentalenolactone biosynthetic process [GO:1901780], (+)-epi-alpha-bisabolol biosynthetic process [GO:1901943] Definition: The chemical reactions and pathways resulting in the formation of sesquiterpenoid compounds, terpenoids with three isoprene units.